polyol metabolic process [GO:0019751] (biological process) References: PMID:30240188 Subtypes: inositol metabolic process [GO:0006020], hexitol metabolic process [GO:0006059], glycerol metabolic process [GO:0006071], GO:0006671, pentitol metabolic process [GO:0019519], diol metabolic process [GO:0034311], inositol phosphate metabolic process [GO:0043647], polyol biosynthetic process [GO:0046173], polyol catabolic process [GO:0046174], GO:0051472, GO:1901128, 2-deoxystreptamine metabolic process [GO:1901742] Also known as: polyhydric alcohol metabolic process, polyol metabolism Relationships: is a type of GO:0006066 Definition: The chemical reactions and pathways involving a polyol, any alcohol containing three or more hydroxyl groups attached to saturated carbon atoms.